{
  "gene": "UniProtKB:P02724",
  "gene_name": "Glycophorin-A",
  "gene_symbol": "GYPA",
  "term_label": "Unknown molecular function",
  "term_id": "UNKNOWN:0001"
}